response to meiotic DNA replication checkpoint signaling [GO:0072441] (biological process) Sources: GOC:mtg_cell_cycle Also known as: meiotic DNA replication checkpoint effector process, response to signal involved in meiotic DNA replication checkpoint Relationships: is a type of GO:0072410; is a type of response to DNA replication checkpoint signaling [GO:0072438] Definition: A process that occurs in response to signals generated as a result of meiotic DNA replication checkpoint signaling.